{
  "term_id": "GO:0006570",
  "gene_name": "Iodotyrosine deiodinase 1",
  "term_label": "tyrosine metabolic process",
  "gene": "UniProtKB:Q6PHW0",
  "gene_symbol": "IYD"
}